{
  "term_label": "Unknown biological process",
  "gene_name": "Protein phosphatase methylesterase 1",
  "gene_symbol": "PPME1",
  "term_id": "UNKNOWN:0002",
  "gene": "UniProtKB:Q9Y570"
}